{
  "gene_name": "Histone H1.1",
  "gene_symbol": "H1-1",
  "term_label": "euchromatin",
  "gene": "UniProtKB:Q02539",
  "term_id": "GO:0000791"
}